ERBB4-ERBB3 complex [GO:0038140] (cellular component) Definition: A heterodimeric complex between the tyrosine kinase receptors ERBB4 (also called HER4) and ERBB3 (also called HER3). ERBB3 has impaired kinase activity so relies on the kinase activity of its heterodimer partner for activation and signal transmission. Relationships: is a type of GO:0098802 Also known as: ERBB3-ERBB4 complex, ERBB4:ERBB3 heterodimer References: PMID:16460914 Sources: GOC:signaling